{
  "term_id": "UNKNOWN:0002",
  "term_label": "Unknown biological process",
  "gene_name": "Myocilin opposite strand protein",
  "gene_symbol": "MYOCOS",
  "gene": "UniProtKB:A0A1B0GUC4"
}